{
  "gene": "UniProtKB:Q06136",
  "term_id": "GO:0006666",
  "term_label": "3-keto-sphinganine metabolic process",
  "gene_name": "3-ketodihydrosphingosine reductase",
  "gene_symbol": "KDSR"
}